regulation of phospholipid metabolic process [GO:1903725] (biological process) Definition: Any process that modulates the frequency, rate or extent of phospholipid metabolic process. References: PMID:10657240 Sources: GOC:TermGenie, GO_REF:0000058 Also known as: regulation of phospholipid metabolism Relationships: is a type of regulation of lipid metabolic process [GO:0019216]; is_a regulation of phosphorus metabolic process [GO:0051174]; regulates phospholipid metabolic process [GO:0006644] Subtypes: regulation of phosphatidylinositol dephosphorylation [GO:0060304], regulation of phospholipid catabolic process [GO:0060696], GO:0071071, GO:0150172, regulation of phosphatidylethanolamine metabolic process [GO:0150175], regulation of cardiolipin metabolic process [GO:1900208], negative regulation of phospholipid metabolic process [GO:1903726], positive regulation of phospholipid metabolic process [GO:1903727]